{
  "gene_name": "Mas-related G-protein coupled receptor member D",
  "gene": "UniProtKB:Q8TDS7",
  "term_id": "GO:0004930",
  "term_label": "G protein-coupled receptor activity",
  "gene_symbol": "MRGPRD"
}